{
  "gene": "UniProtKB:Q6FI81",
  "gene_name": "Anamorsin",
  "term_label": "Unknown molecular function",
  "gene_symbol": "CIAPIN1",
  "term_id": "UNKNOWN:0001"
}